{
  "term_label": "Swr1 complex",
  "gene_name": "DNA methyltransferase 1-associated protein 1",
  "term_id": "GO:0000812",
  "gene_symbol": "DMAP1",
  "gene": "UniProtKB:Q9NPF5"
}